positive regulation of cell proliferation involved in mesonephros development [GO:2000608] (biological process) Relationships: is a type of positive regulation of cell proliferation involved in kidney development [GO:1901724]; is a type of regulation of cell proliferation involved in mesonephros development [GO:2000606]; positively regulates cell proliferation involved in mesonephros development [GO:0061209] Subtypes: GO:2000092 Sources: GOC:obol Definition: Any process that activates or increases the frequency, rate or extent of cell proliferation involved in mesonephros development.